regulation of cardiac muscle cell differentiation [GO:2000725] (biological process) Relationships: is a type of GO:0051153; is a type of regulation of cardiocyte differentiation [GO:1905207]; regulates cardiac muscle cell differentiation [GO:0055007] Also known as: regulation of cardiomyocyte differentiation, regulation of heart muscle cell differentiation Subtypes: regulation of cardiac muscle fiber development [GO:0055018], negative regulation of cardiac muscle cell differentiation [GO:2000726], positive regulation of cardiac muscle cell differentiation [GO:2000727] Definition: Any process that modulates the frequency, rate or extent of cardiac muscle cell differentiation. Sources: GOC:BHF